{
  "term_label": "Unknown biological process",
  "gene": "UniProtKB:Q9H4G4",
  "gene_name": "Golgi-associated plant pathogenesis-related protein 1",
  "term_id": "UNKNOWN:0002",
  "gene_symbol": "GLIPR2"
}